{
  "term_id": "GO:0030182",
  "gene": "UniProtKB:P41225",
  "gene_name": "Transcription factor SOX-3",
  "gene_symbol": "SOX3",
  "term_label": "neuron differentiation"
}